{
  "gene": "UniProtKB:P0C2W1",
  "term_label": "synapse",
  "gene_symbol": "FBXO45",
  "gene_name": "F-box_SPRY domain-containing protein 1",
  "term_id": "GO:0045202"
}